{
  "gene_name": "Sialomucin core protein 24",
  "term_label": "Unknown biological process",
  "gene_symbol": "CD164",
  "gene": "UniProtKB:Q04900",
  "term_id": "UNKNOWN:0002"
}